{
  "gene_name": "Peroxisome proliferator-activated receptor delta",
  "term_label": "RNA polymerase II transcription regulator complex",
  "gene": "UniProtKB:Q03181",
  "term_id": "GO:0090575",
  "gene_symbol": "PPARD"
}